{
  "gene": "UniProtKB:Q96A35",
  "term_id": "GO:0005739",
  "gene_name": "Large ribosomal subunit protein uL24m",
  "term_label": "mitochondrion",
  "gene_symbol": "MRPL24"
}